apo-beta-carotenoid-14',13'-dioxygenase activity [GO:0050588] (molecular function) Relationships: is_a oxidoreductase activity, acting on single donors with incorporation of molecular oxygen, incorporation of one atom of oxygen (internal monooxygenases or internal mixed function oxidases) [GO:0016703] Definition: Catalysis of the reaction: 8'-apo-beta-carotenol + O2 = (E,E)-7-hydroxy-6-methylhepta-3,5-dienal + 14'-apo-beta-carotenal. Also known as: apo-b-carotenoid-14',13'-dioxygenase activity, 8'-apo-beta-carotenol:O2 oxidoreductase activity Sources: EC:1.13.11.67, RHEA:26023